{
  "gene_name": "Homeobox protein Nkx-6.2",
  "term_label": "regulation of transcription by RNA polymerase II",
  "gene_symbol": "NKX6-2",
  "term_id": "GO:0006357",
  "gene": "UniProtKB:Q9C056"
}